positive regulation of plasmacytoid dendritic cell antigen processing and presentation [GO:0002612] (biological process) Sources: GOC:add Definition: Any process that activates or increases the frequency, rate, or extent of plasmacytoid dendritic cell antigen processing and presentation. Relationships: is a type of positive regulation of dendritic cell antigen processing and presentation [GO:0002606]; is a type of regulation of plasmacytoid dendritic cell antigen processing and presentation [GO:0002610]; positively regulates plasmacytoid dendritic cell antigen processing and presentation [GO:0002470] Also known as: up regulation of plasmacytoid dendritic cell antigen processing and presentation, up-regulation of plasmacytoid dendritic cell antigen processing and presentation, upregulation of plasmacytoid dendritic cell antigen processing and presentation, activation of plasmacytoid dendritic cell antigen processing and presentation, stimulation of plasmacytoid dendritic cell antigen processing and presentation